{
  "term_label": "ubiquitin protein ligase activity",
  "term_id": "GO:0061630",
  "gene": "UniProtKB:Q969Q1",
  "gene_symbol": "TRIM63",
  "gene_name": "E3 ubiquitin-protein ligase TRIM63"
}